{
  "gene": "UniProtKB:Q9UMD9",
  "gene_symbol": "COL17A1",
  "term_id": "GO:0030056",
  "gene_name": "Collagen alpha-1(XVII) chain",
  "term_label": "hemidesmosome"
}